{
  "term_id": "GO:2000806",
  "gene_symbol": "PPP1R10",
  "term_label": "positive regulation of termination of RNA polymerase II transcription, poly(A)-coupled",
  "gene": "UniProtKB:Q96QC0",
  "gene_name": "Serine_threonine-protein phosphatase 1 regulatory subunit 10"
}